leukotriene A4 metabolic process [GO:1901751] (biological process) Sources: GOC:TermGenie, GOC:yaf Definition: The chemical reactions and pathways involving leukotriene A4. Relationships: is a type of long-chain fatty acid metabolic process [GO:0001676]; is a type of GO:0006691; is a type of epoxide metabolic process [GO:0097176]; is_a fatty acid derivative metabolic process [GO:1901568] Subtypes: leukotriene A4 catabolic process [GO:1901752], leukotriene A4 biosynthetic process [GO:1901753] Also known as: leukotriene A4 metabolism